clypeo-labral disc morphogenesis [GO:0007453] (biological process) Relationships: is a type of imaginal disc morphogenesis [GO:0007560]; is part of clypeo-labral disc development [GO:0035213] Also known as: clypeo-labral disc metamorphosis, morphogenesis of structures derived from the clypeo-labral disc Sources: GOC:bf, ISBN:0879694238 Definition: The process in which the anatomical structures derived from the clypeo-labral disc are generated and organized. This includes the transformation of a clypeo-labal imaginal disc from a monolayered epithelium in the larvae of holometabolous insects into recognizable adult structures including the labrum, anterior and posterior cibarial plates, fish trap bristles, epistomal sclerite and clypeus.